regulation of L-arginine import across plasma membrane [GO:1905541] (biological process) Also known as: regulation of L-arginine import, regulation of L-arginine import into cell Subtypes: negative regulation of L-arginine import across plasma membrane [GO:1905542], positive regulation of L-arginine import across plasma membrane [GO:1905589] References: PMID:14718525 Sources: GOC:TermGenie, GO_REF:0000058 Definition: Any process that modulates the frequency, rate or extent of L-arginine import across plasma membrane. Relationships: is a type of regulation of amino acid import across plasma membrane [GO:0010958]; is a type of regulation of organic acid transport [GO:0032890]; regulates L-arginine import across plasma membrane [GO:0097638]